{
  "term_label": "cellular response to light stimulus",
  "gene": "UniProtKB:P08100",
  "gene_name": "Rhodopsin",
  "term_id": "GO:0071482",
  "gene_symbol": "RHO"
}